{
  "gene_name": "Collagen alpha-1(XXI) chain",
  "term_label": "Unknown biological process",
  "term_id": "UNKNOWN:0002",
  "gene_symbol": "COL21A1",
  "gene": "UniProtKB:Q96P44"
}